pre-B cell receptor complex [GO:0035369] (cellular component) Definition: An immunoglobulin-like complex that is present in at least the plasma membrane of pre-B cells, and that is composed of two identical immunoglobulin heavy chains and two surrogate light chains, each composed of the lambda-5 and VpreB proteins, and a signaling subunit, a heterodimer of the Ig-alpha and Ig-beta proteins. References: PMID:16464608, PMID:17306522 Sources: GOC:add, ISBN:0781765196 Note: Despite its name, the pre-BCR is not a receptor complex, as it appears to provide a low level of signal not dependent on a ligand, but rather simply on correct assembly of the complex as a measure for correct Ig heavy chain recombination and folding. A significant proportion of pre-BCR complexes fail to reach the cell surface, and in some cases may provide their signaling function from the trans-Golgi network or lysosome. Relationships: is a type of membrane protein complex [GO:0098796] Also known as: pre-BCR